type II hypersensitivity [GO:0002445] (biological process) Sources: GOC:add, ISBN:0781735149 Subtypes: type IIa hypersensitivity [GO:0001794], type IIb hypersensitivity [GO:0001795] Regulation: regulated by regulation of type II hypersensitivity [GO:0002892]; negatively regulated by GO:0002893; RO_0002213 by GO:0002894 Relationships: is a type of GO:0002444; is a type of hypersensitivity [GO:0002524]; is a type of immunoglobulin mediated immune response [GO:0016064] Definition: An inflammatory response resulting in cell death or dysfunction mediated by activation of the classical complement pathway or induction of effector cell phagocytosis, cytolysis mechanisms via complement or Fc receptors following the binding of antibodies to cell surface antigens on a target cell, or mediated by the direct binding of antibody to cellular receptors.